{
  "gene_symbol": "STK26",
  "term_label": "cytoplasm",
  "gene_name": "Serine_threonine-protein kinase 26",
  "term_id": "GO:0005737",
  "gene": "UniProtKB:Q9P289"
}